positive regulation of catalase activity [GO:1902553] (biological process) References: PMID:24285797 Sources: GOC:TermGenie Definition: Any process that activates or increases the frequency, rate or extent of catalase activity. Relationships: is a type of positive regulation of oxidoreductase activity [GO:0051353]; positively regulates catalase activity [GO:0004096] Also known as: positive regulation of caperase activity, positive regulation of catalase reaction, positive regulation of catalase-peroxidase activity, positive regulation of equilase activity, positive regulation of hydrogen-peroxide:hydrogen-peroxide oxidoreductase activity, positive regulation of optidase activity, up regulation of caperase activity, up regulation of catalase activity, up regulation of catalase reaction, up regulation of catalase-peroxidase activity, up regulation of equilase activity, up regulation of hydrogen-peroxide:hydrogen-peroxide oxidoreductase activity, up regulation of optidase activity, up-regulation of caperase activity, up-regulation of catalase activity, up-regulation of catalase reaction, up-regulation of catalase-peroxidase activity, up-regulation of equilase activity, up-regulation of hydrogen-peroxide:hydrogen-peroxide oxidoreductase activity, up-regulation of optidase activity, upregulation of caperase activity, upregulation of catalase activity, upregulation of catalase reaction, upregulation of catalase-peroxidase activity, upregulation of equilase activity, upregulation of hydrogen-peroxide:hydrogen-peroxide oxidoreductase activity, upregulation of optidase activity, activation of bacterial catalase-peroxidase activity, activation of caperase activity, activation of catalase activity, activation of catalase reaction, activation of catalase-peroxidase activity, activation of equilase activity, activation of haem catalase activity, activation of heme catalase activity, activation of hydrogen-peroxide:hydrogen-peroxide oxidoreductase activity, activation of manganese catalase activity, activation of optidase activity, positive regulation of bacterial catalase-peroxidase activity, positive regulation of haem catalase activity, positive regulation of heme catalase activity, positive regulation of manganese catalase activity, up regulation of bacterial catalase-peroxidase activity, up regulation of haem catalase activity, up regulation of heme catalase activity, up regulation of manganese catalase activity, up-regulation of bacterial catalase-peroxidase activity, up-regulation of haem catalase activity, up-regulation of heme catalase activity, up-regulation of manganese catalase activity, upregulation of bacterial catalase-peroxidase activity, upregulation of haem catalase activity, upregulation of heme catalase activity, upregulation of manganese catalase activity, activation of CAT, positive regulation of CAT, up regulation of CAT, up-regulation of CAT, upregulation of CAT